{
  "term_label": "structural constituent of nuclear pore",
  "gene_name": "Nuclear pore complex protein Nup133",
  "gene": "UniProtKB:Q8WUM0",
  "term_id": "GO:0017056",
  "gene_symbol": "NUP133"
}